{
  "term_label": "Unknown molecular function",
  "term_id": "UNKNOWN:0001",
  "gene": "UniProtKB:Q9UQB8",
  "gene_symbol": "BAIAP2",
  "gene_name": "Brain-specific angiogenesis inhibitor 1-associated protein 2"
}